{
  "gene": "UniProtKB:Q9ULK6",
  "gene_symbol": "RNF150",
  "term_id": "GO:0005737",
  "gene_name": "RING finger protein 150",
  "term_label": "cytoplasm"
}